{
  "gene": "UniProtKB:P46779",
  "gene_symbol": "RPL28",
  "term_id": "GO:0022625",
  "gene_name": "Large ribosomal subunit protein eL28",
  "term_label": "cytosolic large ribosomal subunit"
}